{
  "gene": "UniProtKB:Q9Y2D9",
  "term_label": "regulation of transcription by RNA polymerase II",
  "gene_symbol": "ZNF652",
  "gene_name": "Zinc finger protein 652",
  "term_id": "GO:0006357"
}